{
  "gene_symbol": "P2RY14",
  "term_id": "GO:0045028",
  "gene_name": "P2Y purinoceptor 14",
  "term_label": "G protein-coupled purinergic nucleotide receptor activity",
  "gene": "UniProtKB:Q15391"
}